{
  "gene_name": "ATP-dependent RNA helicase DHX8",
  "gene": "UniProtKB:Q14562",
  "term_label": "RNA binding",
  "gene_symbol": "DHX8",
  "term_id": "GO:0003723"
}